negative regulation of mast cell proliferation [GO:0070667] (biological process) Definition: Any process that stops, prevents or reduces the rate or extent of mast cell proliferation. Sources: GOC:add, GOC:mah Also known as: down regulation of mast cell proliferation, down-regulation of mast cell proliferation, downregulation of mast cell proliferation, inhibition of mast cell proliferation Relationships: is_a negative regulation of leukocyte proliferation [GO:0070664]; is a type of regulation of mast cell proliferation [GO:0070666]; RO_0002212 GO:0070662